{
  "gene": "UniProtKB:Q96DU9",
  "gene_name": "Polyadenylate-binding protein 5",
  "gene_symbol": "PABPC5",
  "term_label": "cytosol",
  "term_id": "GO:0005829"
}